{
  "gene": "UniProtKB:Q4L180",
  "gene_symbol": "FILIP1L",
  "term_id": "UNKNOWN:0001",
  "term_label": "Unknown molecular function",
  "gene_name": "Filamin A-interacting protein 1-like"
}